{
  "gene_symbol": "NAPA",
  "term_label": "syntaxin binding",
  "gene": "UniProtKB:P54920",
  "gene_name": "Alpha-soluble NSF attachment protein",
  "term_id": "GO:0019905"
}